{
  "term_label": "ephrin receptor binding",
  "term_id": "GO:0046875",
  "gene": "UniProtKB:P52798",
  "gene_name": "Ephrin-A4",
  "gene_symbol": "EFNA4"
}